endothelial cell fate specification [GO:0060847] (biological process) Relationships: is_a cell fate specification [GO:0001708]; is part of endothelial cell fate commitment [GO:0060839] Subtypes: blood vessel endothelial cell fate specification [GO:0097101] Definition: The process involved in the specification of identity of an endothelial cell. Once specification has taken place, a cell will be committed to differentiate down a specific pathway if left in its normal environment. Sources: GOC:dph, GOC:sdb_2009, GOC:tb